{
  "term_label": "chromatin DNA binding",
  "term_id": "GO:0031490",
  "gene_name": "Histone demethylase UTY",
  "gene": "UniProtKB:O14607",
  "gene_symbol": "UTY"
}